beta-galactosidase activity (lactose isomerization) [GO:0103033] (molecular function) Definition: Catalysis of the reaction: alpha-lactose = beta-(1->6)-galactobiose. Relationships: is a type of intramolecular acyltransferase activity [GO:0016867] Sources: EC:5.4.1.-, GOC:pz